RQC-trigger complex [GO:0180022] (cellular component) Also known as: ASC-1 complex, RQT complex, activating signal cointegrator 1 complex References: PMID:12077347, PMID:28757607, PMID:32099016 Relationships: is a type of protein-containing complex [GO:0032991] Definition: A ribosome disassembly complex which dissociates stalled ribsome subunits as part of the ribosome quality control pathway. RQT complex is composed of a RNA helicase-family protein yeast Rqt2 (human ASCC3), a ubiquitin-binding protein yeast Rqt3, (human ASCC2), and Rqt4 (human TRIP4). The human complex has an additional component protein ASCC1 and can act as a transcriptional coactivator by interacting with transcription factors such as NF-kappa B.